{
  "gene_symbol": "KDM4A",
  "gene": "UniProtKB:O75164",
  "term_id": "GO:0006338",
  "gene_name": "Lysine-specific demethylase 4A",
  "term_label": "chromatin remodeling"
}